{
  "term_label": "retinol metabolic process",
  "gene_symbol": "ADH1A",
  "term_id": "GO:0042572",
  "gene": "UniProtKB:P07327",
  "gene_name": "Alcohol dehydrogenase 1A"
}